{
  "gene_name": "Endoribonuclease Dicer",
  "gene": "UniProtKB:Q9UPY3",
  "term_id": "GO:0005634",
  "term_label": "nucleus",
  "gene_symbol": "DICER1"
}